{
  "term_label": "plasma membrane",
  "gene": "UniProtKB:Q8NG76",
  "term_id": "GO:0005886",
  "gene_symbol": "OR2T33",
  "gene_name": "Olfactory receptor 2T33"
}